{
  "gene": "UniProtKB:Q9HD42",
  "gene_name": "Charged multivesicular body protein 1a",
  "gene_symbol": "CHMP1A",
  "term_label": "ESCRT III complex",
  "term_id": "GO:0000815"
}